{
  "term_label": "triglyceride metabolic process",
  "gene_name": "Glycerol kinase 3",
  "term_id": "GO:0006641",
  "gene_symbol": "GK3",
  "gene": "UniProtKB:Q14409"
}